cell fate specification [GO:0001708] (biological process) Sources: GOC:go_curators Definition: The cellular developmental process involved in cell fate commitment in which the cell is designated to follow a developmental path, unless they receive extrinsic cues that direct an alternative fate. Relationships: is a type of GO:0048869; is part of cell fate commitment [GO:0045165] Regulation: negatively regulated by negative regulation of cell fate specification [GO:0009996]; regulated by regulation of cell fate specification [GO:0042659]; positively regulated by GO:0042660 Subtypes: endodermal cell fate specification [GO:0001714], ectodermal cell fate specification [GO:0001715], GO:0007501, epidermal cell fate specification [GO:0009957], GO:0010158, GO:0010234, GO:0014018, GO:0014817, GO:0021780, GO:0035153, eosinophil fate specification [GO:0035857], compound eye cone cell fate specification [GO:0042679], GO:0042694, myoblast fate specification [GO:0048626], neuron fate specification [GO:0048665], stem cell fate specification [GO:0048866], cell fate specification involved in pattern specification [GO:0060573], GO:0060847, GO:0060912, vulval cell fate specification [GO:0072327], bundle sheath cell fate specification [GO:0090610], plant epidermal cell fate specification [GO:0090628], plant endodermal cell fate specification [GO:0160057]